{
  "term_id": "GO:0005886",
  "gene_symbol": "GUCY2D",
  "term_label": "plasma membrane",
  "gene": "UniProtKB:Q02846",
  "gene_name": "Retinal guanylyl cyclase 1"
}